germ tube [GO:0032179] (cellular component) Relationships: is a type of cellular anatomical structure [GO:0110165] Definition: The slender tubular outgrowth first produced by most spores in germination. Sources: ISBN:0877799148